{
  "term_label": "cytoplasm",
  "gene_name": "Envoplakin",
  "gene": "UniProtKB:Q92817",
  "gene_symbol": "EVPL",
  "term_id": "GO:0005737"
}